{
  "term_label": "Unknown biological process",
  "term_id": "UNKNOWN:0002",
  "gene": "UniProtKB:Q9BVP2",
  "gene_name": "Guanine nucleotide-binding protein-like 3",
  "gene_symbol": "GNL3"
}